{
  "gene_name": "Keratin-associated protein 27-1",
  "term_id": "UNKNOWN:0002",
  "gene": "UniProtKB:Q3LI81",
  "term_label": "Unknown biological process",
  "gene_symbol": "KRTAP27-1"
}